{
  "term_id": "GO:0000149",
  "term_label": "SNARE binding",
  "gene_name": "Vesicle-associated membrane protein 7",
  "gene_symbol": "VAMP7",
  "gene": "UniProtKB:P51809"
}